{
  "term_label": "structural constituent of nuclear pore",
  "term_id": "GO:0017056",
  "gene": "UniProtKB:Q9BW27",
  "gene_name": "Nuclear pore complex protein Nup85",
  "gene_symbol": "NUP85"
}